{
  "gene_symbol": "HSP90AA2P",
  "gene": "UniProtKB:Q14568",
  "term_id": "GO:0051082",
  "term_label": "unfolded protein binding",
  "gene_name": "Heat shock protein HSP 90-alpha A2"
}